{
  "term_id": "GO:0045087",
  "gene": "UniProtKB:Q5W0U4",
  "gene_symbol": "BSPRY",
  "gene_name": "B box and SPRY domain-containing protein",
  "term_label": "innate immune response"
}